{
  "term_id": "GO:0043186",
  "gene_symbol": "MOV10L1",
  "term_label": "P granule",
  "gene_name": "RNA helicase Mov10l1",
  "gene": "UniProtKB:Q9BXT6"
}